regulation of metabolic process [GO:0019222] (biological process) Definition: Any process that modulates the frequency, rate or extent of the chemical reactions and pathways within a cell or an organism. Relationships: is a type of regulation of cellular process [GO:0050794]; regulates metabolic process [GO:0008152] Sources: GOC:go_curators Also known as: regulation of metabolism, regulation of multicellular organismal metabolic process, regulation of organismal metabolic process Subtypes: GO:0009889, negative regulation of metabolic process [GO:0009892], positive regulation of metabolic process [GO:0009893], regulation of catabolic process [GO:0009894], regulation of photosynthesis [GO:0010109], regulation of ketone metabolic process [GO:0010565], regulation of collagen metabolic process [GO:0010712], regulation of hormone metabolic process [GO:0032350], regulation of amine metabolic process [GO:0033238], regulation of amide metabolic process [GO:0034248], regulation of sulfur metabolic process [GO:0042762], regulation of secondary metabolic process [GO:0043455], regulation of generation of precursor metabolites and energy [GO:0043467], regulation of phosphorus metabolic process [GO:0051174], regulation of macromolecule metabolic process [GO:0060255], GO:0060263, GO:0062012, regulation of primary metabolic process [GO:0080090], regulation of nitric oxide metabolic process [GO:0080164], regulation of organohalogen metabolic process [GO:0090347], GO:0120161, regulation of tetrapyrrole metabolic process [GO:1901401], regulation of nitrogen cycle metabolic process [GO:1903314], regulation of bioluminescence [GO:1905085], regulation of oxygen metabolic process [GO:2000374], GO:2000377